phenylacetyl-CoA 1,2-epoxidase activity [GO:0097266] (molecular function) Relationships: is a type of GO:0016709 Also known as: phenylacetyl-CoA epoxidase activity, phenylacetyl-CoA monooxygenase activity, ring 1,2-phenylacetyl-CoA epoxidase activity References: PMID:20660314, PMID:21247899 Sources: EC:1.14.13.149, GOC:bf, GOC:gk Definition: Catalysis of the reaction: phenylacetyl-CoA + H+ + NADPH + O2 = 2-(1,2-epoxy-1,2-dihydrophenyl)acetyl-CoA + H2O + NADP+.